{
  "gene_symbol": "AIRE",
  "gene_name": "Autoimmune regulator",
  "gene": "UniProtKB:O43918",
  "term_label": "negative thymic T cell selection",
  "term_id": "GO:0045060"
}